{
  "gene_symbol": "SLC1A2",
  "term_label": "glutamate:sodium symporter activity",
  "gene_name": "Excitatory amino acid transporter 2",
  "term_id": "GO:0015501",
  "gene": "UniProtKB:P43004"
}